{
  "term_label": "fatty acid catabolic process",
  "gene_symbol": "LPIN1",
  "gene": "UniProtKB:Q14693",
  "term_id": "GO:0009062",
  "gene_name": "Phosphatidate phosphatase LPIN1"
}